{
  "gene_name": "Zinc finger protein 701",
  "gene": "UniProtKB:Q9NV72",
  "term_label": "RNA polymerase II cis-regulatory region sequence-specific DNA binding",
  "gene_symbol": "ZNF701",
  "term_id": "GO:0000978"
}